protein dealkylation [GO:0008214] (biological process) Definition: The removal of an alkyl group from a protein amino acid. Alkyl groups are derived from alkanes by removal of one hydrogen atom. Relationships: is a type of protein modification process [GO:0036211] Also known as: protein amino acid dealkylation Subtypes: protein demethylation [GO:0006482] Sources: GOC:ai